{
  "term_label": "Unknown cellular component",
  "term_id": "UNKNOWN:0003",
  "gene_name": "Zinc finger protein 680",
  "gene_symbol": "ZNF680",
  "gene": "UniProtKB:Q8NEM1"
}